{
  "gene": "UniProtKB:O75712",
  "term_label": "gap junction channel activity",
  "gene_name": "Gap junction beta-3 protein",
  "gene_symbol": "GJB3",
  "term_id": "GO:0005243"
}